{
  "gene_symbol": "TUBGCP3",
  "term_id": "GO:0051321",
  "gene": "UniProtKB:Q96CW5",
  "gene_name": "Gamma-tubulin complex component 3",
  "term_label": "meiotic cell cycle"
}